{
  "gene_symbol": "PNRC2",
  "term_label": "nucleus",
  "gene_name": "Proline-rich nuclear receptor coactivator 2",
  "term_id": "GO:0005634",
  "gene": "UniProtKB:Q9NPJ4"
}